hemidesmosome [GO:0030056] (cellular component) Definition: A cell-substrate junction (attachment structure) found in epithelial cells that links intermediate filaments to extracellular matrices via transmembrane complexes. In vertebrates, hemidesmosomes mediate contact between the basal side of epithelial cells and the basal lamina. In C. elegans, hemidesmosomes connect epithelial cells to distinct extracellular matrices on both the apical and basal cell surfaces. References: PMID:20205195 Sources: GOC:kmv, ISBN:0815316208 Also known as: epidermal attachment structure, fibrous organelle, trans-epithelial attachment, hemi-adherens junction Relationships: is_a cell-substrate junction [GO:0030055]